tube fusion [GO:0035146] (biological process) Definition: The joining of specific branches of a tubular system to form a continuous network. Sources: GOC:bf Relationships: is a type of tube morphogenesis [GO:0035239]; is part of branching morphogenesis of an epithelial tube [GO:0048754] Subtypes: branch fusion, open tracheal system [GO:0035147]